regulation of cargo loading into COPII-coated vesicle [GO:1901301] (biological process) Subtypes: negative regulation of cargo loading into COPII-coated vesicle [GO:1901303] Definition: Any process that modulates the frequency, rate or extent of cargo loading into COPII-coated vesicle. Also known as: regulation of cargo loading into COPII vesicle, regulation of cargo selection into COPII-coated vesicle, regulation of COPII coat-cargo complex assembly References: PMID:15899885 Sources: GOC:TermGenie, GOC:lb Relationships: is a type of GO:0032386; regulates COPII-coated vesicle cargo loading [GO:0090110]